{
  "gene_name": "Tetratricopeptide repeat protein 16",
  "term_label": "Unknown molecular function",
  "term_id": "UNKNOWN:0001",
  "gene": "UniProtKB:Q8NEE8",
  "gene_symbol": "TTC16"
}